{
  "gene": "UniProtKB:P62847",
  "gene_symbol": "RPS24",
  "gene_name": "Small ribosomal subunit protein eS24",
  "term_id": "GO:0022627",
  "term_label": "cytosolic small ribosomal subunit"
}